{
  "gene_name": "Serine_threonine-protein phosphatase 2A 56 kDa regulatory subunit epsilon isoform",
  "gene_symbol": "PPP2R5E",
  "term_id": "GO:0000159",
  "term_label": "protein phosphatase type 2A complex",
  "gene": "UniProtKB:Q16537"
}